positive regulation of CD8-positive, alpha-beta cytotoxic T cell extravasation [GO:2000454] (biological process) Definition: Any process that activates or increases the frequency, rate or extent of CD8-positive, alpha-beta cytotoxic T cell extravasation. Relationships: is a type of positive regulation of CD8-positive, alpha-beta T cell extravasation [GO:2000451]; is a type of regulation of CD8-positive, alpha-beta cytotoxic T cell extravasation [GO:2000452]; positively regulates GO:0035698 Sources: GOC:obol